{
  "gene": "UniProtKB:P27448",
  "term_label": "plasma membrane",
  "gene_symbol": "MARK3",
  "gene_name": "MAP_microtubule affinity-regulating kinase 3",
  "term_id": "GO:0005886"
}